negative regulation of barbed-end actin filament capping [GO:2000813] (biological process) Relationships: is a type of positive regulation of actin filament depolymerization [GO:0030836]; is a type of positive regulation of actin filament polymerization [GO:0030838]; is a type of GO:0051129; is a type of GO:2000812; negatively regulates barbed-end actin filament capping [GO:0051016] Definition: Any process that stops, prevents or reduces the frequency, rate or extent of barbed-end actin filament capping. Also known as: negative regulation of barbed-end F-actin capping activity, negative regulation of barbed-end actin capping activity, negative regulation of plus-end F-actin capping activity, negative regulation of plus-end actin filament capping activity Sources: GOC:BHF